COPII vesicle coating [GO:0048208] (biological process) Definition: The addition of COPII proteins and adaptor proteins to ER membranes during the formation of transport vesicles, forming a vesicle coat. References: PMID:10219233 Sources: GOC:ascb_2009, GOC:dph, GOC:jid, GOC:mah, GOC:tb Also known as: COPII coating of ER-derived vesicle, COPII vesicle coat assembly, COPII vesicle coat formation Relationships: is a type of vesicle coating [GO:0006901]; is a type of GO:0065003; is part of vesicle targeting, rough ER to cis-Golgi [GO:0048207]; is part of COPII-coated vesicle budding [GO:0090114] Regulation: regulated by regulation of COPII vesicle coating [GO:0003400]